{
  "term_id": "GO:0006396",
  "gene_name": "Interferon-stimulated gene 20 kDa protein",
  "term_label": "RNA processing",
  "gene": "UniProtKB:Q96AZ6",
  "gene_symbol": "ISG20"
}